1-alkyl-2-acetylglycerol O-acyltransferase activity [GO:0047167] (molecular function) Relationships: is a type of GO:0008374 Definition: Catalysis of the reaction: 1-O-alkyl-2-acetyl-sn-glycerol + acyl-CoA = 1-O-alkyl-2-acetyl-3-acyl-sn-glycerol + CoA. Sources: EC:2.3.1.125, MetaCyc:2.3.1.125-RXN Also known as: 1-hexadecyl-2-acetylglycerol acyltransferase activity, acyl-CoA:1-O-alkyl-2-acetyl-sn-glycerol O-acyltransferase activity